{
  "gene": "UniProtKB:Q12968",
  "gene_symbol": "NFATC3",
  "term_id": "GO:0000981",
  "term_label": "DNA-binding transcription factor activity, RNA polymerase II-specific",
  "gene_name": "Nuclear factor of activated T-cells, cytoplasmic 3"
}